{
  "gene": "UniProtKB:Q86UD0",
  "gene_name": "Suppressor APC domain-containing protein 2",
  "term_id": "UNKNOWN:0003",
  "term_label": "Unknown cellular component",
  "gene_symbol": "SAPCD2"
}